{
  "gene_symbol": "COPS5",
  "gene": "UniProtKB:Q92905",
  "gene_name": "COP9 signalosome complex subunit 5",
  "term_id": "GO:0019784",
  "term_label": "deNEDDylase activity"
}